{
  "gene": "UniProtKB:Q04771",
  "gene_symbol": "ACVR1",
  "gene_name": "Activin receptor type-1",
  "term_label": "plasma membrane",
  "term_id": "GO:0005886"
}